{
  "term_label": "Unknown molecular function",
  "term_id": "UNKNOWN:0001",
  "gene_name": "Nuclear pore complex-interacting protein family member B11",
  "gene_symbol": "NPIPB11",
  "gene": "UniProtKB:E5RHQ5"
}